{
  "gene": "UniProtKB:Q8IUA7",
  "term_label": "Unknown cellular component",
  "gene_name": "ATP-binding cassette sub-family A member 9",
  "term_id": "UNKNOWN:0003",
  "gene_symbol": "ABCA9"
}